{
  "gene_symbol": "DEFA3",
  "term_label": "defense response to Gram-positive bacterium",
  "gene": "UniProtKB:P59666",
  "gene_name": "Neutrophil defensin 3",
  "term_id": "GO:0050830"
}